{
  "term_id": "UNKNOWN:0001",
  "gene": "UniProtKB:Q6ZN18",
  "term_label": "Unknown molecular function",
  "gene_name": "Zinc finger protein AEBP2",
  "gene_symbol": "AEBP2"
}